{
  "gene_symbol": "CST9LP1",
  "gene": "UniProtKB:Q5W188",
  "gene_name": "Putative cystatin-9-like protein CST9LP1",
  "term_label": "Unknown molecular function",
  "term_id": "UNKNOWN:0001"
}